{
  "gene_name": "Diacylglycerol kinase beta",
  "term_label": "ATP-dependent diacylglycerol kinase activity",
  "gene_symbol": "DGKB",
  "term_id": "GO:0004143",
  "gene": "UniProtKB:Q9Y6T7"
}